{
  "term_label": "positive regulation of transcription by RNA polymerase II",
  "gene_name": "Transcription factor AP-2 gamma",
  "gene_symbol": "TFAP2C",
  "gene": "UniProtKB:Q92754",
  "term_id": "GO:0045944"
}